{
  "gene_name": "Myocyte-specific enhancer factor 2C",
  "term_label": "Unknown cellular component",
  "term_id": "UNKNOWN:0003",
  "gene_symbol": "MEF2C",
  "gene": "UniProtKB:Q06413"
}